protein demalonylation [GO:0036046] (BP) Subtypes: peptidyl-lysine demalonylation [GO:0036047] References: PMID:22076378 Sources: GOC:sp Relationships: is a type of protein deacylation [GO:0035601] Definition: The removal of a malonyl group (CO-CH2-CO), from an amino acid residue within a protein or peptide.